{
  "gene": "UniProtKB:Q14147",
  "gene_name": "Probable ATP-dependent RNA helicase DHX34",
  "gene_symbol": "DHX34",
  "term_id": "GO:0000184",
  "term_label": "nuclear-transcribed mRNA catabolic process, nonsense-mediated decay"
}